positive regulation of ascospore-type prospore membrane formation [GO:1903024] (biological process) References: PMID:11405625 Sources: GOC:TermGenie, GO_REF:0000058 Relationships: is a type of positive regulation of cellular component biogenesis [GO:0044089]; is a type of positive regulation of cellular component organization [GO:0051130]; is a type of positive regulation of ascospore formation [GO:0075296]; is a type of regulation of ascospore-type prospore membrane formation [GO:1903023]; positively regulates GO:0032120 Also known as: positive regulation of FSM assembly, positive regulation of FSM biosynthesis, positive regulation of FSM formation, positive regulation of forespore membrane biosynthesis, positive regulation of forespore membrane formation, up regulation of FSM assembly, up regulation of FSM biosynthesis, up regulation of FSM formation, up regulation of ascospore-type prospore membrane assembly, up regulation of forespore membrane biosynthesis, up regulation of forespore membrane formation, up-regulation of FSM assembly, up-regulation of FSM biosynthesis, up-regulation of FSM formation, up-regulation of ascospore-type prospore membrane assembly, up-regulation of forespore membrane biosynthesis, up-regulation of forespore membrane formation, upregulation of FSM assembly, upregulation of FSM biosynthesis, upregulation of FSM formation, upregulation of ascospore-type prospore membrane assembly, upregulation of forespore membrane biosynthesis, upregulation of forespore membrane formation, activation of FSM assembly, activation of FSM biosynthesis, activation of FSM formation, activation of ascospore-type prospore membrane assembly, activation of forespore membrane biosynthesis, activation of forespore membrane formation, positive regulation of ascospore-type prospore membrane assembly Definition: Any process that activates or increases the frequency, rate or extent of formation of an ascospore-type prospore membrane.